{
  "gene_symbol": "BCAS4",
  "gene_name": "Breast carcinoma-amplified sequence 4",
  "term_label": "Unknown molecular function",
  "gene": "UniProtKB:Q8TDM0",
  "term_id": "UNKNOWN:0001"
}